{
  "gene_symbol": "SLC27A1",
  "gene_name": "Long-chain fatty acid transport protein 1",
  "gene": "UniProtKB:Q6PCB7",
  "term_id": "GO:0005886",
  "term_label": "plasma membrane"
}